{
  "term_label": "glycerophosphodiester phosphodiesterase activity",
  "term_id": "GO:0008889",
  "gene": "UniProtKB:Q9HCC8",
  "gene_name": "Glycerophosphoinositol inositolphosphodiesterase GDPD2",
  "gene_symbol": "GDPD2"
}